D-arabinonolactonase activity [GO:0047815] (molecular function) Sources: EC:3.1.1.30, RHEA:23108 Also known as: D-arabinono-1,4-lactone lactonohydrolase activity Relationships: is a type of carboxylic ester hydrolase activity [GO:0052689] Definition: Catalysis of the reaction: D-arabinono-1,4-lactone + H2O = D-arabinonate + H+.